dGMP biosynthetic process [GO:0006181] (biological process) Also known as: dGMP anabolism, dGMP biosynthesis, dGMP formation, dGMP synthesis Relationships: is a type of purine deoxyribonucleotide biosynthetic process [GO:0009153]; is a type of GO:0009171; is a type of GO:0046054 Sources: ISBN:0198506732 Definition: The chemical reactions and pathways resulting in the formation of dGMP, deoxyguanosine monophosphate (2'-deoxyguanosine 5'-phosphate). Subtypes: dGMP salvage [GO:0106384]